Sertoli cell proliferation [GO:0060011] (biological process) Relationships: is a type of GO:0050673; BFO_0000050 GO:0008584 Sources: GOC:dph Definition: The multiplication or reproduction of Sertoli cells, resulting in the expansion of the Sertoli cell population. A Sertoli cell is a supporting cell projecting inward from the basement membrane of seminiferous tubules.